cellular response to gravity [GO:0071258] (biological process) Also known as: cellular response to gravitational stimulus Sources: GOC:mah Relationships: is a type of response to gravity [GO:0009629]; is a type of cellular response to abiotic stimulus [GO:0071214] Definition: Any process that results in a change in state or activity of a cell (in terms of movement, secretion, enzyme production, gene expression, etc.) as a result of a gravitational stimulus.